{
  "term_id": "GO:0032580",
  "term_label": "Golgi cisterna membrane",
  "gene": "UniProtKB:A8MQT2",
  "gene_name": "Golgin subfamily A member 8B",
  "gene_symbol": "GOLGA8B"
}